translocation of peptides or proteins into symbiont [GO:0051844] (biological process) Relationships: is a type of translocation of molecules into symbiont [GO:0051862] Definition: The directed movement of peptides or proteins produced by an organism to a location inside the symbiont organism. The symbiont is defined as the smaller of the organisms involved in a symbiotic interaction. Sources: GOC:cc Also known as: transport of peptides or proteins into symbiont